{
  "gene_name": "Melanoma-associated antigen B3",
  "gene_symbol": "MAGEB3",
  "term_label": "Unknown molecular function",
  "term_id": "UNKNOWN:0001",
  "gene": "UniProtKB:O15480"
}